pyridoxal phosphatase activity [GO:0033883] (molecular function) Definition: Catalysis of the reaction: pyridoxal 5'-phosphate + H2O = pyridoxal + phosphate. Relationships: is a type of phosphatase activity [GO:0016791] Also known as: vitamin B6 (pyridoxine) phosphatase activity, vitamin B6-phosphate phosphatase activity, PLP phosphatase activity, PNP phosphatase activity, pyridoxal-5'-phosphate phosphohydrolase activity Sources: EC:3.1.3.74